{
  "term_id": "GO:0005212",
  "gene_symbol": "CRYGA",
  "term_label": "structural constituent of eye lens",
  "gene_name": "Gamma-crystallin A",
  "gene": "UniProtKB:P11844"
}